{
  "gene_symbol": "RND2",
  "term_label": "signal transduction",
  "gene": "UniProtKB:P52198",
  "term_id": "GO:0007165",
  "gene_name": "Rho-related GTP-binding protein RhoN"
}